{
  "term_label": "Unknown molecular function",
  "gene_name": "Protein SREK1IP1",
  "gene": "UniProtKB:Q8N9Q2",
  "gene_symbol": "SREK1IP1",
  "term_id": "UNKNOWN:0001"
}